{
  "gene_name": "Receptor tyrosine-protein kinase erbB-3",
  "gene": "UniProtKB:P21860",
  "term_id": "GO:0050679",
  "term_label": "positive regulation of epithelial cell proliferation",
  "gene_symbol": "ERBB3"
}